negative regulation of basophil differentiation [GO:0045641] (biological process) Definition: Any process that stops, prevents, or reduces the frequency, rate or extent of basophil differentiation. Sources: GOC:go_curators Also known as: down regulation of basophil differentiation, down-regulation of basophil differentiation, downregulation of basophil differentiation, inhibition of basophil differentiation Relationships: is_a negative regulation of granulocyte differentiation [GO:0030853]; is a type of regulation of basophil differentiation [GO:0045640]; negatively regulates basophil differentiation [GO:0030221]